regulation of cell-cell adhesion mediated by cadherin [GO:2000047] (biological process) Definition: Any process that modulates the frequency, rate or extent of cell-cell adhesion mediated by cadherin. Sources: GOC:obol Relationships: is a type of regulation of cell-cell adhesion [GO:0022407]; regulates cell-cell adhesion mediated by cadherin [GO:0044331] Subtypes: GO:2000048, positive regulation of cell-cell adhesion mediated by cadherin [GO:2000049]